{
  "term_id": "UNKNOWN:0002",
  "term_label": "Unknown biological process",
  "gene": "UniProtKB:Q6NZ63",
  "gene_symbol": "STEAP1B",
  "gene_name": "STEAP family member 1B"
}